glucose 1-phosphate metabolic process [GO:0019255] (biological process) Subtypes: glucose 1-phosphate phosphorylation [GO:0006009] Sources: GOC:ai Relationships: is a type of GO:0006796; is a type of organophosphate metabolic process [GO:0019637]; is a type of GO:1901135 Definition: The chemical reactions and pathways involving glucose 1-phosphate, a monophosphorylated derivative of glucose with the phosphate group attached to C-1. Also known as: glucose 1-phosphate metabolism, glucose 1-phosphate utilization